{
  "term_id": "GO:0008168",
  "gene_symbol": "NSUN4",
  "term_label": "methyltransferase activity",
  "gene_name": "5-methylcytosine rRNA methyltransferase NSUN4",
  "gene": "UniProtKB:Q96CB9"
}